{
  "gene": "UniProtKB:Q15043",
  "term_label": "plasma membrane",
  "gene_name": "Metal cation symporter ZIP14",
  "gene_symbol": "SLC39A14",
  "term_id": "GO:0005886"
}